{
  "gene_name": "ATPase GET3",
  "term_id": "GO:0016887",
  "gene": "UniProtKB:O43681",
  "gene_symbol": "GET3",
  "term_label": "ATP hydrolysis activity"
}